{
  "term_label": "neuronal cell body",
  "gene_symbol": "COBL",
  "gene_name": "Protein cordon-bleu",
  "term_id": "GO:0043025",
  "gene": "UniProtKB:O75128"
}